{
  "gene_symbol": "LRRC1",
  "term_label": "cytoplasm",
  "gene_name": "Leucine-rich repeat-containing protein 1",
  "term_id": "GO:0005737",
  "gene": "UniProtKB:Q9BTT6"
}